{
  "term_id": "GO:0005737",
  "gene_name": "M-phase inducer phosphatase 1",
  "term_label": "cytoplasm",
  "gene": "UniProtKB:P30304",
  "gene_symbol": "CDC25A"
}